{
  "gene_name": "Putative uncharacterized protein FLJ43944",
  "term_id": "UNKNOWN:0001",
  "term_label": "Unknown molecular function",
  "gene_symbol": "Q6ZRG5",
  "gene": "UniProtKB:Q6ZRG5"
}